{
  "gene_symbol": "TP53",
  "term_label": "regulation of apoptotic process",
  "term_id": "GO:0042981",
  "gene_name": "Cellular tumor antigen p53",
  "gene": "UniProtKB:P04637"
}